{
  "gene_symbol": "KLRC1",
  "gene_name": "NKG2-A_NKG2-B type II integral membrane protein",
  "gene": "UniProtKB:P26715",
  "term_label": "stimulatory C-type lectin receptor signaling pathway",
  "term_id": "GO:0002223"
}